{
  "term_id": "UNKNOWN:0002",
  "gene": "UniProtKB:Q96II8",
  "gene_name": "DISP complex protein LRCH3",
  "term_label": "Unknown biological process",
  "gene_symbol": "LRCH3"
}